head kidney formation [GO:0072117] (biological process) Relationships: is a type of pronephros formation [GO:0072116]; is part of GO:0072115 Sources: GOC:mtg_kidney_jan10, ZFA:0000669 Definition: The developmental process pertaining to the initial formation of the head kidney. The head kidney is a pronephros that consists of fused bilateral lobes located in the anterior part of the kidney.